{
  "term_id": "GO:0006954",
  "gene_symbol": "CCL1",
  "gene": "UniProtKB:P22362",
  "gene_name": "C-C motif chemokine 1",
  "term_label": "inflammatory response"
}